{
  "gene_symbol": "TMEM119",
  "gene_name": "Transmembrane protein 119",
  "term_id": "GO:0033690",
  "gene": "UniProtKB:Q4V9L6",
  "term_label": "positive regulation of osteoblast proliferation"
}